{
  "term_label": "plasma membrane",
  "term_id": "GO:0005886",
  "gene_name": "Olfactory receptor 2C1",
  "gene_symbol": "OR2C1",
  "gene": "UniProtKB:O95371"
}